ciliary transition zone [GO:0035869] (cellular component) Also known as: cilial transition zone, cilium transition zone, connecting cilium Subtypes: photoreceptor connecting cilium [GO:0032391] Relationships: is a type of cellular anatomical structure [GO:0110165]; is part of cilium [GO:0005929] References: PMID:21422230 Sources: GOC:cilia, GOC:kmv Note: Depending on the species, this region may have a distinct geometrically shaped electron-dense structure within the axonemal lumen visible in electron microscopy images; most animals don't display this inner structure. The axoneme extends through the ciliary transition zone, but only consists of the outer doublets. The central pair, axonemal spokes, and dynein complexes are not found in this part of the ciliary shaft. Note that the connecting cilium of the photoreceptor cells is thought to be equivalent to the transition zone. Definition: A region of the cilium between the basal body and proximal segment that is characterized by Y-shaped assemblages that connect axonemal microtubules to the ciliary membrane. The ciliary transition zone appears to function as a gate that controls ciliary membrane composition and separates the cytosol from the ciliary plasm.